{
  "gene_symbol": "ACTG1",
  "gene": "UniProtKB:P63261",
  "term_id": "GO:0005737",
  "gene_name": "Actin, cytoplasmic 2",
  "term_label": "cytoplasm"
}